{
  "term_id": "UNKNOWN:0003",
  "gene_name": "Ubiquitin domain-containing protein TINCR",
  "gene": "UniProtKB:A0A2R8Y7D0",
  "term_label": "Unknown cellular component",
  "gene_symbol": "TINCR"
}